{
  "term_label": "transcription cis-regulatory region binding",
  "gene_name": "Ankyrin repeat domain-containing protein 23",
  "term_id": "GO:0000976",
  "gene": "UniProtKB:Q86SG2",
  "gene_symbol": "ANKRD23"
}